{
  "term_label": "Unknown cellular component",
  "gene_symbol": "MAPDA",
  "gene": "UniProtKB:Q6DHV7",
  "term_id": "UNKNOWN:0003",
  "gene_name": "Adenosine deaminase-like protein"
}